{
  "gene": "UniProtKB:Q9HCI5",
  "gene_name": "Melanoma-associated antigen E1",
  "gene_symbol": "MAGEE1",
  "term_id": "GO:0000122",
  "term_label": "negative regulation of transcription by RNA polymerase II"
}